{
  "gene_name": "G-protein coupled receptor 143",
  "term_label": "G protein-coupled receptor signaling pathway",
  "gene": "UniProtKB:P51810",
  "gene_symbol": "GPR143",
  "term_id": "GO:0007186"
}